mesonephric macula densa development [GO:0061220] (biological process) Relationships: is a type of mesonephric nephron epithelium development [GO:0061241]; is a type of macula densa development [GO:0072024]; is part of mesonephric juxtaglomerular apparatus development [GO:0061212] Sources: GOC:mtg_kidney_jan10 Definition: The process whose specific outcome is the progression of the mesonephric macula densa over time, from its formation to the mature structure. The mesonephric macula densa is an area of specialized cells in the distal tubule of the mesonephros that makes contact with the vascular pole of the glomerulus.